unconventional myosin complex [GO:0016461] (cellular component) Relationships: is a type of myosin complex [GO:0016459] Subtypes: myosin IV complex [GO:0031474], myosin V complex [GO:0031475], myosin VI complex [GO:0031476], GO:0031477, myosin VIII complex [GO:0031478], GO:0031479, myosin X complex [GO:0031480], GO:0031481, myosin XII complex [GO:0031482], myosin XIII complex [GO:0031483], myosin XIV complex [GO:0031484], GO:0031485, myosin XVI complex [GO:0031486], myosin XVII complex [GO:0031487], myosin XVIII complex [GO:0031488], myosin III complex [GO:0042385], myosin I complex [GO:0045160] Definition: A portmanteau term for myosins other than myosin II. Sources: GOC:ma Note: Note that this term is retained because it is widely used by biologists. Also known as: non-muscle myosin